{
  "gene_symbol": "MEOX1",
  "gene": "UniProtKB:P50221",
  "gene_name": "Homeobox protein MOX-1",
  "term_label": "somite development",
  "term_id": "GO:0061053"
}